cellular response to ergosterol [GO:1901625] (biological process) Relationships: is a type of cellular response to sterol [GO:0036315]; is a type of GO:0097306 Sources: GOC:TermGenie Definition: Any process that results in a change in state or activity of a cell (in terms of movement, secretion, enzyme production, gene expression, etc.) as a result of an ergosterol stimulus.